{
  "term_label": "response to nicotine",
  "gene_symbol": "CHRNA3",
  "gene_name": "Neuronal acetylcholine receptor subunit alpha-3",
  "term_id": "GO:0035094",
  "gene": "UniProtKB:P32297"
}